{
  "gene": "UniProtKB:Q7RTY7",
  "term_label": "Unknown cellular component",
  "gene_symbol": "OVCH1",
  "gene_name": "Ovochymase-1",
  "term_id": "UNKNOWN:0003"
}